negative regulation of heat generation [GO:0031651] (biological process) Definition: Any process that stops, prevents, or reduces the rate or extent of heat generation. Sources: GOC:dph, GOC:mah, GOC:tb Subtypes: negative regulation of fever generation [GO:0031621] Also known as: down regulation of heat generation, down-regulation of heat generation, downregulation of heat generation, inhibition of heat generation Relationships: is a type of regulation of heat generation [GO:0031650]; is a type of GO:0051241; negatively regulates heat generation [GO:0031649]